{
  "term_label": "RNA polymerase II cis-regulatory region sequence-specific DNA binding",
  "gene": "UniProtKB:O15015",
  "term_id": "GO:0000978",
  "gene_name": "Zinc finger protein 646",
  "gene_symbol": "ZNF646"
}